{
  "gene_name": "Solute carrier family 35 member C2",
  "term_label": "antiporter activity",
  "term_id": "GO:0015297",
  "gene": "UniProtKB:Q9NQQ7",
  "gene_symbol": "SLC35C2"
}